{
  "term_label": "Cul4-RING E3 ubiquitin ligase complex",
  "gene_name": "DDB1- and CUL4-associated factor 12-like protein 2",
  "gene_symbol": "DCAF12L2",
  "term_id": "GO:0080008",
  "gene": "UniProtKB:Q5VW00"
}